{
  "gene_name": "Immunoglobulin kappa variable 1-39",
  "term_id": "GO:0006955",
  "gene_symbol": "IGKV1-39",
  "gene": "UniProtKB:P01597",
  "term_label": "immune response"
}